external side of plasma membrane [GO:0009897] (cellular component) Subtypes: periplasmic side of plasma membrane [GO:0098567], external side of apical plasma membrane [GO:0098591] Definition: The leaflet of the plasma membrane that faces away from the cytoplasm and any proteins embedded or anchored in it or attached to its surface. Also known as: juxtamembrane, external leaflet of plasma membrane, outer surface of cytoplasmic membrane Sources: GOC:dos, GOC:tb Relationships: is a type of side of membrane [GO:0098552]; is part of GO:0005886; is part of GO:0009986